{
  "gene": "UniProtKB:P55318",
  "gene_symbol": "FOXA3",
  "term_label": "cell differentiation",
  "term_id": "GO:0030154",
  "gene_name": "Hepatocyte nuclear factor 3-gamma"
}